{
  "term_label": "bone mineralization involved in bone maturation",
  "gene": "UniProtKB:A6NI56",
  "gene_symbol": "CCDC154",
  "term_id": "GO:0035630",
  "gene_name": "Coiled-coil domain-containing protein 154"
}